{
  "term_label": "cadherin binding",
  "gene_name": "Cadherin-6",
  "gene": "UniProtKB:P55285",
  "term_id": "GO:0045296",
  "gene_symbol": "CDH6"
}